{
  "term_label": "Unknown molecular function",
  "gene_symbol": "LINC00299",
  "gene_name": "Putative uncharacterized protein encoded by LINC00299",
  "gene": "UniProtKB:Q6ZSB3",
  "term_id": "UNKNOWN:0001"
}